negative regulation of anaphase-promoting complex-dependent catabolic process [GO:1905785] (biological process) Definition: Any process that stops, prevents or reduces the frequency, rate or extent of anaphase-promoting complex-dependent catabolic process. References: PMID:10921876 Sources: GOC:TermGenie, GO_REF:0000058 Relationships: is a type of negative regulation of proteasomal ubiquitin-dependent protein catabolic process [GO:0032435]; is a type of GO:1905784; negatively regulates anaphase-promoting complex-dependent catabolic process [GO:0031145]